{
  "term_label": "nuclear membrane",
  "gene": "UniProtKB:Q8IXM6",
  "term_id": "GO:0031965",
  "gene_symbol": "NRM",
  "gene_name": "Nurim"
}